lncRNA-mediated post-transcriptional gene silencing [GO:0000512] (biological process) Note: This term should be applied to lncRNAs and proteins associated with this process and not to the target (miRNAs or mRNAs) of the process. Relationships: is_a GO:0035194 Definition: A post-transcriptional gene silencing pathway in which regulatory long noncoding RNAs (lncRNAs) elicit silencing of specific target genes, often miRNAs or mRNAs. Also known as: lncRNA-mediated gene silencing References: PMID:34454184, PMID:35055152